{
  "gene": "UniProtKB:Q9NX78",
  "term_id": "UNKNOWN:0003",
  "gene_symbol": "TMEM260",
  "gene_name": "Transmembrane protein 260",
  "term_label": "Unknown cellular component"
}